mRNA 3'-UTR binding [GO:0003730] (molecular function) Sources: GOC:mah Relationships: is a type of mRNA binding [GO:0003729] Definition: Binding to a 3' untranslated region of an mRNA molecule. Subtypes: mRNA 3'-UTR AU-rich region binding [GO:0035925] Also known as: mRNA 3' UTR binding